{
  "term_id": "GO:0015630",
  "gene_name": "MAP7 domain-containing protein 1",
  "gene_symbol": "MAP7D1",
  "term_label": "microtubule cytoskeleton",
  "gene": "UniProtKB:Q3KQU3"
}